{
  "gene_name": "Cell division cycle protein 16 homolog",
  "gene": "UniProtKB:Q13042",
  "term_label": "anaphase-promoting complex-dependent catabolic process",
  "term_id": "GO:0031145",
  "gene_symbol": "CDC16"
}